3-isopropylmalate dehydrogenase activity [GO:0003862] (molecular function) Also known as: (2R,3S)-3-isopropylmalate:NAD+ oxidoreductase activity, 3-carboxy-2-hydroxy-4-methylpentanoate:NAD+ oxidoreductase activity, IMDH activity, IPMDH, beta-IPM dehydrogenase activity, beta-isopropylmalate dehydrogenase activity, beta-isopropylmalic enzyme, threo-Ds-3-isopropylmalate dehydrogenase activity Definition: Catalysis of the reaction: (2R,3S)-3-isopropylmalate + NAD+ = 4-methyl-2-oxopentanoate + CO2 + NADH. Sources: RHEA:32271 Relationships: is_a oxidoreductase activity, acting on the CH-OH group of donors, NAD or NADP as acceptor [GO:0016616]